{
  "term_id": "GO:0005131",
  "term_label": "growth hormone receptor binding",
  "gene_symbol": "GH2",
  "gene": "UniProtKB:P01242",
  "gene_name": "Growth hormone variant"
}